neutral lipid metabolic process [GO:0006638] (biological process) Also known as: neutral lipid metabolism Relationships: is a type of lipid metabolic process [GO:0006629] Definition: The chemical reactions and pathways involving neutral lipids, lipids only soluble in solvents of very low polarity. Subtypes: GO:0006639, neutral lipid biosynthetic process [GO:0046460], neutral lipid catabolic process [GO:0046461] Sources: ISBN:0198547684